hydrogen dehydrogenase activity [GO:0047985] (molecular function) Also known as: bidirectional hydrogenase activity, hydrogenase activity, H(2):NAD(+) oxidoreductase activity, H2:NAD+ oxidoreductase activity, NAD-linked hydrogenase activity, hydrogen:NAD+ oxidoreductase activity Relationships: is a type of oxidoreductase activity, acting on hydrogen as donor, NAD or NADP as acceptor [GO:0016696] Sources: EC:1.12.1.2, MetaCyc:HYDROGEN-DEHYDROGENASE-RXN Definition: Catalysis of the reaction: H2 + NAD+ = H+ + NADH.